{
  "term_id": "UNKNOWN:0001",
  "gene_symbol": "A0A1W2PR80",
  "gene": "UniProtKB:A0A1W2PR80",
  "gene_name": "POM121-like protein 1",
  "term_label": "Unknown molecular function"
}